{
  "gene_symbol": "RSBN1",
  "term_label": "histone H4K20 demethylase activity",
  "gene": "UniProtKB:Q5VWQ0",
  "term_id": "GO:0035575",
  "gene_name": "Lysine-specific demethylase 9"
}